positive regulation of acute inflammatory response to non-antigenic stimulus [GO:0002879] (biological process) Sources: GOC:add Definition: Any process that activates or increases the frequency, rate, or extent of an acute inflammatory response to a non-antigenic stimulus. Relationships: is a type of positive regulation of acute inflammatory response [GO:0002675]; is a type of GO:0002877; positively regulates acute inflammatory response to non-antigenic stimulus [GO:0002525] Also known as: up regulation of acute inflammatory response to non-antigenic stimulus, up-regulation of acute inflammatory response to non-antigenic stimulus, upregulation of acute inflammatory response to non-antigenic stimulus, activation of acute inflammatory response to non-antigenic stimulus, stimulation of acute inflammatory response to non-antigenic stimulus